{
  "term_id": "GO:0032049",
  "gene": "UniProtKB:Q32NB8",
  "term_label": "cardiolipin biosynthetic process",
  "gene_symbol": "PGS1",
  "gene_name": "CDP-diacylglycerol--glycerol-3-phosphate 3-phosphatidyltransferase, mitochondrial"
}